{
  "term_id": "GO:0005634",
  "term_label": "nucleus",
  "gene": "UniProtKB:Q96KQ7",
  "gene_name": "Histone-lysine N-methyltransferase EHMT2",
  "gene_symbol": "EHMT2"
}